{
  "term_label": "mitotic spindle assembly",
  "term_id": "GO:0090307",
  "gene_name": "Kinesin-like protein KIF11",
  "gene_symbol": "KIF11",
  "gene": "UniProtKB:P52732"
}